positive regulation of protein transport [GO:0051222] (biological process) Definition: Any process that activates or increases the frequency, rate or extent of the directed movement of a protein into, out of or within a cell, or between cells, by means of some agent such as a transporter or pore. Subtypes: GO:0042998, positive regulation of protein secretion [GO:0050714], positive regulation of intracellular protein transport [GO:0090316], positive regulation of lipoprotein transport [GO:0140077], positive regulation of protein import into chloroplast stroma [GO:1904216], GO:1904591, positive regulation of ubiquitin-dependent endocytosis [GO:2000397] Sources: GOC:ai Relationships: is a type of GO:0051050; is a type of regulation of protein transport [GO:0051223]; is_a positive regulation of protein localization [GO:1903829]; is a type of GO:1904951; positively regulates GO:0015031 Also known as: up regulation of protein transport, up-regulation of protein transport, upregulation of protein transport, activation of protein transport, stimulation of protein transport